response to spindle assembly checkpoint signaling [GO:0072485] (biological process) Definition: A process that occurs in response to signals generated as a result of spindle assembly checkpoint signaling. Sources: GOC:mtg_cell_cycle Also known as: response to signal involved in spindle assembly checkpoint, spindle assembly checkpoint effector process Subtypes: GO:0072464, response to mitotic cell cycle spindle assembly checkpoint signaling [GO:0072479] Relationships: is a type of response to spindle checkpoint signaling [GO:0072417]